{
  "gene_name": "Probable ATP-dependent RNA helicase DDX4",
  "term_label": "germ cell development",
  "gene_symbol": "DDX4",
  "term_id": "GO:0007281",
  "gene": "UniProtKB:Q9NQI0"
}